{
  "term_id": "GO:0005886",
  "gene_symbol": "GRAMD1C",
  "gene_name": "Protein Aster-C",
  "gene": "UniProtKB:Q8IYS0",
  "term_label": "plasma membrane"
}